{
  "term_id": "UNKNOWN:0003",
  "gene_symbol": "TMEM249",
  "gene_name": "Cation channel sperm-associated auxiliary subunit TMEM249",
  "gene": "UniProtKB:Q2WGJ8",
  "term_label": "Unknown cellular component"
}